{
  "gene_name": "Threonylcarbamoyl-AMP synthase",
  "term_label": "tRNA binding",
  "term_id": "GO:0000049",
  "gene_symbol": "YRDC",
  "gene": "UniProtKB:Q86U90"
}